{
  "term_label": "structural constituent of eye lens",
  "term_id": "GO:0005212",
  "gene_name": "Gamma-crystallin B",
  "gene_symbol": "CRYGB",
  "gene": "UniProtKB:P07316"
}